phosphatidylserine flippase activity [GO:0140346] (molecular function) References: PMID:11870854 Relationships: is_a aminophospholipid flippase activity [GO:0015247]; is a type of glycerophospholipid flippase activity [GO:0140333] Also known as: phosphatidylserine flippase activity (exoplasmic to cytosolic leaflet) Definition: Catalysis of the movement of phosphatidylserine from the exoplasmic to the cytosolic leaflet of a membrane, using energy from the hydrolysis of ATP.